carbon utilization [GO:0015976] (biological process) Definition: A series of processes that forms an integrated mechanism by which a cell or an organism detects the depletion of primary carbon sources and then activates genes to scavenge the last traces of the primary carbon source and to transport and metabolize alternative carbon sources such as carbon dioxide or carbonic acid. The utilization process begins when the cell or organism detects carbon levels, includes the activation of genes whose products detect, transport or metabolize carbon-containing substances, and ends when carbon is incorporated into the cell or organism's metabolism. Sources: GOC:mah, GOC:mlg Also known as: carbon utilization by utilization of organic compounds, heterotrophy Relationships: is a type of response to nutrient levels [GO:0031667] Regulation: regulated by regulation of carbon utilization [GO:0043609]